{
  "term_id": "UNKNOWN:0001",
  "gene_name": "Protein FAM27D1",
  "gene": "UniProtKB:Q5T7N8",
  "term_label": "Unknown molecular function",
  "gene_symbol": "FAM27D1"
}